{
  "term_id": "GO:0001676",
  "gene_name": "Long-chain fatty acid transport protein 3",
  "term_label": "long-chain fatty acid metabolic process",
  "gene_symbol": "SLC27A3",
  "gene": "UniProtKB:Q5K4L6"
}